{
  "gene_symbol": "SGO2",
  "term_id": "GO:0030892",
  "gene": "UniProtKB:Q562F6",
  "gene_name": "Shugoshin 2",
  "term_label": "mitotic cohesin complex"
}